{
  "gene": "UniProtKB:Q9Y4F3",
  "term_id": "UNKNOWN:0002",
  "gene_name": "Meiosis regulator and mRNA stability factor 1",
  "gene_symbol": "MARF1",
  "term_label": "Unknown biological process"
}